{
  "gene": "UniProtKB:Q9H8N7",
  "gene_name": "Zinc finger protein 395",
  "gene_symbol": "ZNF395",
  "term_id": "GO:0000978",
  "term_label": "RNA polymerase II cis-regulatory region sequence-specific DNA binding"
}